cardiac atrium development [GO:0003230] (biological process) Definition: The process whose specific outcome is the progression of a cardiac atrium over time, from its formation to the mature structure. A cardiac atrium receives blood from a vein and pumps it to a cardiac ventricle. Relationships: is a type of cardiac chamber development [GO:0003205] Sources: GOC:mtg_heart